{
  "gene": "UniProtKB:P04156",
  "term_id": "GO:0005886",
  "gene_symbol": "PRNP",
  "term_label": "plasma membrane",
  "gene_name": "Major prion protein"
}